{
  "gene_symbol": "TAS2R4",
  "term_label": "membrane",
  "gene_name": "Taste receptor type 2 member 4",
  "term_id": "GO:0016020",
  "gene": "UniProtKB:Q9NYW5"
}